{
  "term_label": "Unknown molecular function",
  "term_id": "UNKNOWN:0001",
  "gene_name": "X-ray radiation resistance-associated protein 1",
  "gene": "UniProtKB:Q6P2D8",
  "gene_symbol": "XRRA1"
}